{
  "gene": "UniProtKB:Q6P582",
  "gene_symbol": "MZT2A",
  "term_id": "GO:0005813",
  "gene_name": "Mitotic-spindle organizing protein 2A",
  "term_label": "centrosome"
}